dextran 1,6-alpha-isomaltotriosidase activity [GO:0033924] (molecular function) Definition: Catalysis of the hydrolysis of (1->6)-alpha-D-glucosidic linkages in dextrans, to remove successive isomaltotriose units from the non-reducing ends of the chains. Also known as: 1,6-alpha-D-glucan isomaltotriohydrolase activity, exo-isomaltotriohydrolase activity Relationships: is a type of hydrolase activity, hydrolyzing O-glycosyl compounds [GO:0004553] Sources: EC:3.2.1.95